{
  "term_label": "Unknown molecular function",
  "gene": "UniProtKB:Q6ZRX8",
  "term_id": "UNKNOWN:0001",
  "gene_name": "Putative uncharacterized protein FLJ45999",
  "gene_symbol": "Q6ZRX8"
}